{
  "gene": "UniProtKB:Q96QV1",
  "gene_symbol": "HHIP",
  "term_label": "Unknown biological process",
  "gene_name": "Hedgehog-interacting protein",
  "term_id": "UNKNOWN:0002"
}